{
  "term_label": "Set1C/COMPASS complex",
  "gene_name": "WD repeat-containing protein 5",
  "term_id": "GO:0048188",
  "gene": "UniProtKB:P61964",
  "gene_symbol": "WDR5"
}